{
  "term_label": "chloride transmembrane transport",
  "term_id": "GO:1902476",
  "gene_name": "Gamma-aminobutyric acid receptor subunit alpha-2",
  "gene": "UniProtKB:P47869",
  "gene_symbol": "GABRA2"
}